negative regulation of CD4-positive, alpha-beta T cell activation [GO:2000515] (biological process) Subtypes: negative regulation of CD4-positive, alpha-beta T cell differentiation [GO:0043371], GO:2000518, negative regulation of CD4-positive, alpha-beta T cell proliferation [GO:2000562] Sources: GOC:obol Definition: Any process that stops, prevents or reduces the frequency, rate or extent of CD4-positive, alpha-beta T cell activation. Relationships: is a type of negative regulation of alpha-beta T cell activation [GO:0046636]; is a type of regulation of CD4-positive, alpha-beta T cell activation [GO:2000514]; negatively regulates CD4-positive, alpha-beta T cell activation [GO:0035710]